{
  "gene_name": "E3 ubiquitin-protein ligase RNF128",
  "gene_symbol": "RNF128",
  "term_id": "GO:0006511",
  "gene": "UniProtKB:Q8TEB7",
  "term_label": "ubiquitin-dependent protein catabolic process"
}